rRNA acetylation [GO:1990882] (biological process) Definition: The modification of rRNA structure by addition of an acetyl group to rRNA. An acetyl group is CH3CO-, derived from acetic [ethanoic] acid. Subtypes: rRNA acetylation involved in maturation of SSU-rRNA [GO:1904812] Relationships: is a type of rRNA modification [GO:0000154]; is a type of RNA acetylation [GO:1990884] References: PMID:25402480